depyrimidination [GO:0045008] (biological process) Definition: The disruption of the bond between the sugar in the backbone and the C or T base, causing the base to be removed and leaving a depyrimidinated sugar. Relationships: is a type of base-excision repair, AP site formation [GO:0006285]; is a type of DNA modification [GO:0006304]; is a type of pyrimidine deoxyribonucleotide catabolic process [GO:0009223] Sources: GOC:ai